{
  "gene_name": "Olfactory receptor 51G1",
  "gene": "UniProtKB:Q8NGK1",
  "term_label": "plasma membrane",
  "gene_symbol": "OR51G1",
  "term_id": "GO:0005886"
}